{
  "gene_name": "Ankyrin repeat and LEM domain-containing protein 1",
  "gene": "UniProtKB:Q8NAG6",
  "term_label": "cytoplasm",
  "term_id": "GO:0005737",
  "gene_symbol": "ANKLE1"
}